{
  "term_label": "protein polyubiquitination",
  "gene_symbol": "UBE2QL1",
  "term_id": "GO:0000209",
  "gene_name": "Ubiquitin-conjugating enzyme E2Q-like protein 1",
  "gene": "UniProtKB:A1L167"
}